{
  "gene": "UniProtKB:P45378",
  "term_label": "troponin complex",
  "gene_name": "Troponin T, fast skeletal muscle",
  "gene_symbol": "TNNT3",
  "term_id": "GO:0005861"
}